{
  "gene": "UniProtKB:Q14181",
  "term_label": "Unknown molecular function",
  "gene_name": "DNA polymerase alpha subunit B",
  "term_id": "UNKNOWN:0001",
  "gene_symbol": "POLA2"
}